{
  "term_id": "GO:0045271",
  "term_label": "respiratory chain complex I",
  "gene": "UniProtKB:P56556",
  "gene_name": "NADH dehydrogenase [ubiquinone] 1 alpha subcomplex subunit 6",
  "gene_symbol": "NDUFA6"
}